{
  "gene": "UniProtKB:P22792",
  "gene_name": "Carboxypeptidase N subunit 2",
  "gene_symbol": "CPN2",
  "term_id": "UNKNOWN:0002",
  "term_label": "Unknown biological process"
}